{
  "term_label": "Unknown cellular component",
  "gene_name": "Thioredoxin domain-containing protein 16",
  "gene_symbol": "TXNDC16",
  "gene": "UniProtKB:Q9P2K2",
  "term_id": "UNKNOWN:0003"
}